regulation of maltoheptaose transport [GO:1900306] (biological process) Definition: Any process that modulates the frequency, rate or extent of maltoheptaose transport. Sources: GOC:TermGenie, GOC:mengo_curators Relationships: is a type of regulation of heptasaccharide transport [GO:1900294]; regulates maltoheptaose transport [GO:2001105] Subtypes: GO:1900307, positive regulation of maltoheptaose transport [GO:1900308]